negative regulation of lipid catabolic process [GO:0050995] (biological process) Relationships: is a type of GO:0009895; is a type of GO:0045833; is a type of GO:0050994; negatively regulates GO:0016042 Also known as: down regulation of lipid catabolic process, down-regulation of lipid catabolic process, downregulation of lipid catabolic process, negative regulation of lipid breakdown, negative regulation of lipid catabolism, negative regulation of lipid degradation, inhibition of lipid catabolic process Sources: GOC:ai Subtypes: negative regulation of triglyceride catabolic process [GO:0010897], GO:0010900, negative regulation of glucocorticoid catabolic process [GO:0031950], negative regulation of fatty acid beta-oxidation [GO:0031999], negative regulation of juvenile hormone catabolic process [GO:0045970], GO:0106394, GO:1900498, negative regulation of butyryl-CoA catabolic process to butyrate [GO:1900501], negative regulation of 1-phosphatidyl-1D-myo-inositol 4,5-bisphosphate catabolic process [GO:1902642], negative regulation of prostaglandin catabolic process [GO:1905829] Definition: Any process that stops, prevents, or reduces the frequency, rate or extent of the chemical reactions and pathways resulting in the breakdown of lipids.